{
  "term_id": "UNKNOWN:0001",
  "gene_symbol": "TRBJ2-6",
  "term_label": "Unknown molecular function",
  "gene": "UniProtKB:A0A0A0MT70",
  "gene_name": "T cell receptor beta joining 2-6"
}